{
  "gene": "UniProtKB:A0A590UK24",
  "gene_symbol": "LOC122319696",
  "term_id": "UNKNOWN:0003",
  "term_label": "Unknown cellular component",
  "gene_name": "Uncharacterized protein"
}